{
  "gene_symbol": "PLXNC1",
  "term_label": "positive regulation of axonogenesis",
  "term_id": "GO:0050772",
  "gene_name": "Plexin-C1",
  "gene": "UniProtKB:O60486"
}